{
  "term_label": "MAP kinase kinase kinase activity",
  "gene": "UniProtKB:P15056",
  "gene_name": "Serine_threonine-protein kinase B-raf",
  "gene_symbol": "BRAF",
  "term_id": "GO:0004709"
}